{
  "term_id": "GO:0048245",
  "gene_name": "C-C motif chemokine 25",
  "gene": "UniProtKB:O15444",
  "term_label": "eosinophil chemotaxis",
  "gene_symbol": "CCL25"
}